{
  "gene_name": "Signal peptide peptidase-like 2C",
  "term_label": "membrane protein proteolysis",
  "gene": "UniProtKB:Q8IUH8",
  "gene_symbol": "SPPL2C",
  "term_id": "GO:0033619"
}